{
  "term_label": "nucleus",
  "term_id": "GO:0005634",
  "gene": "UniProtKB:Q16520",
  "gene_name": "Basic leucine zipper transcriptional factor ATF-like",
  "gene_symbol": "BATF"
}